{
  "gene_name": "Zinc finger protein 654",
  "gene_symbol": "ZNF654",
  "term_id": "GO:0000981",
  "gene": "UniProtKB:Q8IZM8",
  "term_label": "DNA-binding transcription factor activity, RNA polymerase II-specific"
}